{
  "term_id": "UNKNOWN:0003",
  "term_label": "Unknown cellular component",
  "gene_symbol": "C12orf56",
  "gene_name": "Uncharacterized protein C12orf56",
  "gene": "UniProtKB:Q8IXR9"
}